adaptation of signaling pathway [GO:0023058] (biological process) Relationships: is_a GO:0009966 Definition: The regulation of a signal transduction pathway in response to a stimulus upon prolonged exposure to that stimulus. Sources: GOC:mtg_signal Also known as: adaptation of signalling pathway Subtypes: GO:0000754, negative adaptation of signaling pathway [GO:0022401], positive adaptation of signaling pathway [GO:0023059]